{
  "gene_symbol": "FCRL4",
  "term_label": "transmembrane signaling receptor activity",
  "gene": "UniProtKB:Q96PJ5",
  "gene_name": "Fc receptor-like protein 4",
  "term_id": "GO:0004888"
}